{
  "term_id": "GO:0051879",
  "gene_name": "Tetratricopeptide repeat protein 4",
  "gene": "UniProtKB:O95801",
  "gene_symbol": "TTC4",
  "term_label": "Hsp90 protein binding"
}